cyclohexanone monooxygenase activity [GO:0018667] (molecular function) Definition: Catalysis of the reaction: cyclohexanone + NADPH + H+ + O2 = 6-hexanolide + NADP+ + H2O. Relationships: is a type of oxidoreductase activity, acting on paired donors, with incorporation or reduction of molecular oxygen, NAD(P)H as one donor, and incorporation of one atom of oxygen [GO:0016709] Also known as: cyclohexanone 1,2-monooxygenase activity, cyclohexanone oxygenase activity, cyclohexanone:NADPH:oxygen oxidoreductase (6-hydroxylating, 1,2-lactonizing) activity, cyclohexanone:NADPH:oxygen oxidoreductase (lactone-forming) Sources: EC:1.14.13.22